negative regulation of mitotic cytokinesis [GO:1902413] (biological process) Definition: Any process that stops, prevents or reduces the frequency, rate or extent of mitotic cytokinesis. Sources: GOC:TermGenie, GOC:mtg_cell_cycle Also known as: down regulation of cytokinesis after mitosis, down regulation of mitotic cytokinesis, down-regulation of cytokinesis after mitosis, down-regulation of mitotic cytokinesis, downregulation of cytokinesis after mitosis, downregulation of mitotic cytokinesis, negative regulation of cytokinesis after mitosis, inhibition of cytokinesis after mitosis, inhibition of mitotic cytokinesis Relationships: is a type of negative regulation of cytokinesis [GO:0032466]; is a type of regulation of mitotic cytokinesis [GO:1902412]; negatively regulates mitotic cytokinesis [GO:0000281] Subtypes: negative regulation of mitotic cytokinetic process [GO:1903437]